pyruvyltransferase activity [GO:0046919] (molecular function) Relationships: is a type of GO:0016747 Definition: Catalysis of the transfer of a pyruvyl (oxopropanoyl) group from one compound to another. Sources: GOC:ai